{
  "term_id": "GO:0007189",
  "gene_symbol": "CRHR1",
  "gene": "UniProtKB:P34998",
  "term_label": "adenylate cyclase-activating G protein-coupled receptor signaling pathway",
  "gene_name": "Corticotropin-releasing factor receptor 1"
}